{
  "gene_name": "Kelch domain-containing protein 8B",
  "gene": "UniProtKB:Q8IXV7",
  "term_label": "cellularization cleavage furrow",
  "gene_symbol": "KLHDC8B",
  "term_id": "GO:0110070"
}